{
  "gene": "UniProtKB:Q6JBY9",
  "gene_symbol": "RCSD1",
  "term_id": "GO:0051015",
  "term_label": "actin filament binding",
  "gene_name": "CapZ-interacting protein"
}